{
  "gene_symbol": "SLC30A5",
  "term_label": "Golgi apparatus",
  "gene": "UniProtKB:Q8TAD4",
  "term_id": "GO:0005794",
  "gene_name": "Proton-coupled zinc antiporter SLC30A5"
}